{
  "gene": "UniProtKB:Q86VW1",
  "term_label": "organic cation transport",
  "gene_name": "Solute carrier family 22 member 16",
  "term_id": "GO:0015695",
  "gene_symbol": "SLC22A16"
}